{
  "gene": "UniProtKB:P63027",
  "gene_name": "Vesicle-associated membrane protein 2",
  "term_label": "plasma membrane",
  "term_id": "GO:0005886",
  "gene_symbol": "VAMP2"
}